jasmonic acid and ethylene-dependent systemic resistance, jasmonic acid mediated signaling pathway [GO:0009868] (biological process) Definition: The series of molecular signals mediated by jasmonic acid involved in jasmonic acid/ethylene (ethene) dependent systemic resistance. Also known as: jasmonic acid and ethene-dependent systemic resistance, jasmonic acid mediated signaling pathway, jasmonic acid mediated signaling pathway (jasmonic acid/ethene-dependent systemic resistance), jasmonic acid mediated signaling pathway (jasmonic acid/ethylene-dependent systemic resistance), jasmonic acid/ethene-dependent systemic resistance, jasmonic acid mediated signaling pathway, jasmonic acid/ethene-dependent systemic resistance, jasmonic acid mediated signalling pathway, jasmonic acid/ethylene-dependent systemic resistance, jasmonic acid mediated signaling pathway, jasmonic acid/ethylene-dependent systemic resistance, jasmonic acid mediated signalling pathway Relationships: is_a GO:0009867; BFO_0000050 response to jasmonic acid stimulus involved in jasmonic acid and ethylene-dependent systemic resistance [GO:0032260] Sources: GOC:jy